{
  "gene_name": "Golgin subfamily A member 6-like protein 7",
  "term_id": "UNKNOWN:0002",
  "gene_symbol": "GOLGA6L7",
  "term_label": "Unknown biological process",
  "gene": "UniProtKB:A0A1B0GV03"
}